{
  "term_label": "Unknown molecular function",
  "gene_name": "Protein canopy homolog 1",
  "gene_symbol": "CNPY1",
  "term_id": "UNKNOWN:0001",
  "gene": "UniProtKB:Q3B7I2"
}